plastid PEP RNA polymerase core enzyme binding [GO:0001052] (molecular function) Relationships: is a type of GO:0001000 References: PMID:20701995 Sources: GOC:txnOH Definition: Binding to a bacterial-type plastid PEP RNA polymerase core enzyme, typically consisting of two alpha, one beta, one beta prime, and one double prime subunit.